negative regulation of glycogen catabolic process [GO:0045818] (BP) Sources: GOC:go_curators Also known as: down regulation of glycogen catabolic process, down-regulation of glycogen catabolic process, downregulation of glycogen catabolic process, negative regulation of glycogen breakdown, negative regulation of glycogen catabolism, negative regulation of glycogen degradation, negative regulation of glycogenolysis, inhibition of glycogen catabolic process Relationships: is_a GO:0005981; is a type of negative regulation of catabolic process [GO:0009895]; is a type of negative regulation of glycogen metabolic process [GO:0070874]; negatively regulates glycogen catabolic process [GO:0005980] Definition: Any process that stops, prevents, or reduces the frequency, rate or extent of the chemical reactions and pathways resulting in the breakdown of glycogen.